{
  "gene": "UniProtKB:Q9NQ76",
  "term_id": "GO:0031214",
  "gene_symbol": "MEPE",
  "gene_name": "Matrix extracellular phosphoglycoprotein",
  "term_label": "biomineral tissue development"
}